{
  "gene_symbol": "TTYH1",
  "gene": "UniProtKB:Q9H313",
  "gene_name": "Protein tweety homolog 1",
  "term_label": "intracellularly calcium-gated chloride channel activity",
  "term_id": "GO:0005229"
}